{
  "gene": "UniProtKB:Q8TE73",
  "gene_symbol": "DNAH5",
  "term_label": "cilium movement involved in cell motility",
  "term_id": "GO:0060294",
  "gene_name": "Dynein axonemal heavy chain 5"
}